{
  "gene_symbol": "UBE3A",
  "gene": "UniProtKB:Q05086",
  "term_label": "regulation of ubiquitin-dependent protein catabolic process",
  "gene_name": "Ubiquitin-protein ligase E3A",
  "term_id": "GO:2000058"
}